{
  "gene": "UniProtKB:Q15466",
  "gene_name": "Nuclear receptor subfamily 0 group B member 2",
  "term_id": "GO:0032922",
  "term_label": "circadian regulation of gene expression",
  "gene_symbol": "NR0B2"
}